{
  "gene": "UniProtKB:P22059",
  "term_id": "GO:0005829",
  "gene_name": "Oxysterol-binding protein 1",
  "term_label": "cytosol",
  "gene_symbol": "OSBP"
}